{
  "gene_symbol": "CYB5R1",
  "term_label": "cytochrome-b5 reductase activity, acting on NAD(P)H",
  "gene_name": "NADH-cytochrome b5 reductase 1",
  "gene": "UniProtKB:Q9UHQ9",
  "term_id": "GO:0004128"
}